response to phylloquinone [GO:0032573] (biological process) Subtypes: cellular response to phylloquinone [GO:0071309] Also known as: response to vitamin K1 Sources: GOC:sl Relationships: is a type of response to vitamin K [GO:0032571] Definition: Any process that results in a change in state or activity of a cell or an organism (in terms of movement, secretion, enzyme production, gene expression, etc.) as a result of a phylloquinone (vitamin K1) stimulus.